{
  "gene_symbol": "IHH",
  "gene_name": "Indian hedgehog protein",
  "term_label": "calcium ion binding",
  "term_id": "GO:0005509",
  "gene": "UniProtKB:Q14623"
}